{
  "term_label": "positive regulation of G1/S transition of mitotic cell cycle",
  "gene": "UniProtKB:P30281",
  "term_id": "GO:1900087",
  "gene_name": "G1_S-specific cyclin-D3",
  "gene_symbol": "CCND3"
}